{
  "term_id": "GO:0004180",
  "gene": "UniProtKB:Q9Y3Q0",
  "term_label": "carboxypeptidase activity",
  "gene_symbol": "NAALAD2",
  "gene_name": "N-acetylated-alpha-linked acidic dipeptidase 2"
}